lactoferrin receptor activity [GO:0033568] (molecular function) Relationships: is a type of cargo receptor activity [GO:0038024] Definition: Combining with lactoferrin and delivering lactoferrin into the cell via endocytosis. Lactoferrin is an iron-binding glycoprotein which binds ferric iron most efficiently at low pH. References: PMID:16261254 Sources: GOC:bf, GOC:mlg